thyroid-stimulating hormone-secreting cell development [GO:0060130] (biological process) Definition: The process whose specific outcome is the progression of a thyroid-stimulating hormone-secreting cell over time, from its formation to the mature structure. A thyroid-stimulating hormone-secreting cell is a basophil cell of the anterior pituitary that produces thyroid stimulating hormone, thyrotrophin. Also known as: TSH-secreting cell development, beta-basophil development, thyroid stimulating hormone secreting cell development, thyrotrope development, thyrotroph development Sources: GOC:dph Relationships: is a type of glandular epithelial cell development [GO:0002068]; is a type of GO:0021884; is part of thyroid-stimulating hormone-secreting cell differentiation [GO:0060129]